{
  "gene_symbol": "ERFL",
  "term_label": "DNA-binding transcription factor activity, RNA polymerase II-specific",
  "term_id": "GO:0000981",
  "gene": "UniProtKB:A0A1W2PQ73",
  "gene_name": "ETS domain-containing transcription factor ERF-like"
}